focal adhesion disassembly [GO:0120181] (biological process) References: PMID:25490267 Relationships: is a type of GO:0120180 Regulation: regulated by GO:0120182; positively regulated by positive regulation of focal adhesion disassembly [GO:0120183]; negatively regulated by negative regulation of focal adhesion disassembly [GO:0120184] Definition: The disaggregation of a focal adhesion into its constituent components. A focal adhesion is a complex of intracellular signaling and structural proteins that provides a structural link between the internal actin cytoskeleton and the ECM, and also functions as a locus of signal transduction activity.